{
  "gene_name": "Histone deacetylase complex subunit SAP18",
  "gene": "UniProtKB:O00422",
  "term_label": "negative regulation of DNA-templated transcription",
  "term_id": "GO:0045892",
  "gene_symbol": "SAP18"
}